{
  "gene_symbol": "CNKSR3",
  "gene": "UniProtKB:Q6P9H4",
  "term_label": "enzyme-linked receptor protein signaling pathway",
  "term_id": "GO:0007167",
  "gene_name": "Connector enhancer of kinase suppressor of ras 3"
}